{
  "gene": "UniProtKB:O60404",
  "gene_symbol": "OR10H3",
  "term_label": "olfactory receptor activity",
  "term_id": "GO:0004984",
  "gene_name": "Olfactory receptor 10H3"
}